{
  "gene": "UniProtKB:P42574",
  "term_label": "neuron differentiation",
  "gene_name": "Caspase-3",
  "term_id": "GO:0030182",
  "gene_symbol": "CASP3"
}